{
  "gene_symbol": "ITPR2",
  "term_id": "GO:0070679",
  "gene": "UniProtKB:Q14571",
  "gene_name": "Inositol 1,4,5-trisphosphate receptor type 2",
  "term_label": "inositol 1,4,5 trisphosphate binding"
}